{
  "term_id": "GO:0030877",
  "gene_name": "Beta-catenin-interacting protein 1",
  "gene": "UniProtKB:Q9NSA3",
  "term_label": "beta-catenin destruction complex",
  "gene_symbol": "CTNNBIP1"
}